{
  "gene_symbol": "PDCL3",
  "term_id": "GO:0001525",
  "gene_name": "Phosducin-like protein 3",
  "gene": "UniProtKB:Q9H2J4",
  "term_label": "angiogenesis"
}